{
  "gene_name": "Krueppel-like factor 10",
  "term_id": "GO:0005634",
  "gene": "UniProtKB:Q13118",
  "gene_symbol": "KLF10",
  "term_label": "nucleus"
}